{
  "term_label": "response to bacterium",
  "gene_name": "T cell receptor alpha variable 1-2",
  "gene": "UniProtKB:A0A0B4J238",
  "gene_symbol": "TRAV1-2",
  "term_id": "GO:0009617"
}